{
  "gene": "UniProtKB:P26992",
  "gene_symbol": "CNTFR",
  "term_label": "interleukin-11 binding",
  "term_id": "GO:0019970",
  "gene_name": "Ciliary neurotrophic factor receptor subunit alpha"
}